{
  "term_id": "GO:0034271",
  "gene_name": "Beclin-1",
  "term_label": "phosphatidylinositol 3-kinase complex, class III, type I",
  "gene_symbol": "BECN1",
  "gene": "UniProtKB:Q14457"
}